{
  "term_label": "transcription coactivator activity",
  "term_id": "GO:0003713",
  "gene_symbol": "MED13",
  "gene": "UniProtKB:Q9UHV7",
  "gene_name": "Mediator of RNA polymerase II transcription subunit 13"
}